{
  "gene_name": "Deformed epidermal autoregulatory factor 1 homolog",
  "gene_symbol": "DEAF1",
  "gene": "UniProtKB:O75398",
  "term_label": "DNA-binding transcription factor activity, RNA polymerase II-specific",
  "term_id": "GO:0000981"
}